{
  "term_id": "UNKNOWN:0002",
  "term_label": "Unknown biological process",
  "gene_name": "Chemokine-like protein TAFA-2",
  "gene": "UniProtKB:Q8N3H0",
  "gene_symbol": "TAFA2"
}